17-alpha,20-alpha-dihydroxypregn-4-en-3-one dehydrogenase [NAD(P)+] activity [GO:0047006] (molecular function) Sources: EC:1.1.1.149 Relationships: is a type of steroid dehydrogenase activity, acting on the CH-OH group of donors, NAD or NADP as acceptor [GO:0033764] Also known as: 20alpha-hydroxy steroid dehydrogenase activity, 20alpha-hydroxysteroid dehydrogenase, 20alpha-hydroxysteroid:NAD(P)+ 20-oxidoreductase activity, 17-alpha,20-alpha-dihydroxypregn-4-en-3-one dehydrogenase activity, 20alpha-HSD, 20alpha-HSDH Definition: Catalysis of the reaction: NAD(P)+ + 17-alpha,20-alpha-dihydroxypregn-4-en-3-one = NAD(P)H + H+ + 17-alpha-hydroxyprogesterone.